{
  "term_id": "GO:0045892",
  "term_label": "negative regulation of DNA-templated transcription",
  "gene": "UniProtKB:Q719H9",
  "gene_symbol": "KCTD1",
  "gene_name": "BTB_POZ domain-containing protein KCTD1"
}